Norrin signaling pathway [GO:0110135] (biological process) Definition: The series of molecular signals initiated by binding of the cysteine knot protein Norrin to a Frizzled 4 (Fzd4) family receptor on the surface of the target cell and ending with a change in cell state. References: PMID:15035989, PMID:17955262 Sources: GOC:BHF, GOC:rl Relationships: is a type of cell surface receptor signaling pathway [GO:0007166]